{
  "term_id": "GO:0043488",
  "gene": "UniProtKB:Q9Y534",
  "gene_name": "Cold shock domain-containing protein C2",
  "gene_symbol": "CSDC2",
  "term_label": "regulation of mRNA stability"
}